{
  "gene_symbol": "FAM13B",
  "term_id": "UNKNOWN:0002",
  "gene_name": "Protein FAM13B",
  "gene": "UniProtKB:Q9NYF5",
  "term_label": "Unknown biological process"
}